{
  "gene_name": "Homeobox protein Hox-D3",
  "gene": "UniProtKB:P31249",
  "term_id": "GO:0000978",
  "term_label": "RNA polymerase II cis-regulatory region sequence-specific DNA binding",
  "gene_symbol": "HOXD3"
}